{
  "term_label": "negative regulation of intracellular estrogen receptor signaling pathway",
  "gene": "UniProtKB:Q13033",
  "gene_name": "Striatin-3",
  "gene_symbol": "STRN3",
  "term_id": "GO:0033147"
}